cellular response to osmotic stress [GO:0071470] (biological process) Definition: Any process that results in a change in state or activity of a cell (in terms of movement, secretion, enzyme production, gene expression, etc.) as a result of a stimulus indicating an increase or decrease in the concentration of solutes outside the organism or cell. Sources: GOC:mah Also known as: cellular osmotic response, cellular osmotic stress response Relationships: is a type of response to osmotic stress [GO:0006970]; is a type of cellular response to chemical stress [GO:0062197]; is_a cellular response to abiotic stimulus [GO:0071214] Subtypes: osmosensory signaling pathway [GO:0007231], intrinsic apoptotic signaling pathway in response to osmotic stress [GO:0008627], cellular response to non-ionic osmotic stress [GO:0071471], cellular response to salt stress [GO:0071472], GO:0071474, cellular hypotonic response [GO:0071476] Regulation: regulated by regulation of cellular response to osmotic stress [GO:0106049]